{
  "gene_name": "Putative protein RFPL3S",
  "gene_symbol": "RFPL3S",
  "term_label": "Unknown biological process",
  "gene": "UniProtKB:P0C7P2",
  "term_id": "UNKNOWN:0002"
}